{
  "gene_symbol": "LY86",
  "gene": "UniProtKB:O95711",
  "term_label": "Unknown cellular component",
  "term_id": "UNKNOWN:0003",
  "gene_name": "Lymphocyte antigen 86"
}